{
  "gene_symbol": "CPNE3",
  "term_id": "GO:0005886",
  "gene": "UniProtKB:O75131",
  "term_label": "plasma membrane",
  "gene_name": "Copine-3"
}